{
  "term_label": "olfactory receptor activity",
  "term_id": "GO:0004984",
  "gene": "UniProtKB:Q6IF36",
  "gene_name": "Putative olfactory receptor 8G2",
  "gene_symbol": "OR8G2P"
}